{
  "gene": "UniProtKB:Q9NR00",
  "term_label": "cytosol",
  "term_id": "GO:0005829",
  "gene_symbol": "TCIM",
  "gene_name": "Transcriptional and immune response regulator"
}